meiotic telomere tethering at nuclear periphery [GO:0044821] (biological process) Definition: The process in which a telomere is maintained in a specific location at the nuclear periphery, as part of a meiotic cell cycle. Sources: GOC:mtg_cell_cycle Relationships: is a type of GO:0034398; is a type of meiotic telomere clustering [GO:0045141]